{
  "term_label": "positive regulation of canonical NF-kappaB signal transduction",
  "gene_name": "Nucleotide-binding oligomerization domain-containing protein 1",
  "gene_symbol": "NOD1",
  "term_id": "GO:0043123",
  "gene": "UniProtKB:Q9Y239"
}